{
  "gene": "UniProtKB:P0C5K6",
  "gene_name": "Putative tumor antigen NA88-A",
  "term_label": "Unknown biological process",
  "gene_symbol": "VENTXP1",
  "term_id": "UNKNOWN:0002"
}